spermatid differentiation [GO:0048515] (biological process) Relationships: is a type of developmental process involved in reproduction [GO:0003006]; is a type of cellular process involved in reproduction in multicellular organism [GO:0022412]; is a type of cell differentiation [GO:0030154]; is part of spermatogenesis [GO:0007283] Also known as: spermatid cell differentiation Sources: GOC:dph, GOC:jid Definition: The process whose specific outcome is the progression of a spermatid over time, from initial commitment of the cell to a specific fate, to the fully functional differentiated cell.